glycerol-3-phosphate 1-dehydrogenase (NADP+) activity [GO:0047014] (molecular function) Also known as: L-glycerol 3-phosphate:NADP oxidoreductase activity, NADPH-dependent glycerin-3-phosphate dehydrogenase activity, glycerin-3-phosphate dehydrogenase activity, glycerol phosphate (nicotinamide adenine dinucleotide phosphate) dehydrogenase activity, sn-glycerol-3-phosphate:NADP+ 1-oxidoreductase activity Sources: RHEA:19773 Relationships: is a type of oxidoreductase activity, acting on the CH-OH group of donors, NAD or NADP as acceptor [GO:0016616] Definition: Catalysis of the reaction: sn-glycerol 3-phosphate + NADP+ = D-glyceraldehyde 3-phosphate + H+ + NADPH.